{
  "gene_name": "Cilia- and flagella-associated protein 58",
  "term_id": "UNKNOWN:0001",
  "term_label": "Unknown molecular function",
  "gene": "UniProtKB:Q5T655",
  "gene_symbol": "CFAP58"
}